response to mycophenolic acid [GO:0071505] (biological process) Relationships: is a type of response to oxygen-containing compound [GO:1901700] Subtypes: GO:0071506 Also known as: response to mycophenolate Definition: Any process that results in a change in state or activity of a cell or an organism (in terms of movement, secretion, enzyme production, gene expression, etc.) as a result of a mycophenolic acid stimulus. Sources: GOC:mah, GOC:yaf